tRNA-dihydrouridine20 synthase activity [GO:0102264] (molecular function) Relationships: is_a tRNA dihydrouridine synthase activity [GO:0017150] Sources: EC:1.3.1.91, GOC:pz Definition: Catalysis of the reaction: a 5,6-dihydrouracil20 in tRNA + NAD(P) = H+ + a uracil20 in tRNA + NAD(P)H.